{
  "gene_name": "Putative tripartite motif-containing protein 64B",
  "gene": "UniProtKB:A6NI03",
  "gene_symbol": "TRIM64B",
  "term_label": "cytoplasm",
  "term_id": "GO:0005737"
}